inositol phosphorylceramide mannosyltransferase activity [GO:0103064] (molecular function) Sources: GOC:pz, RHEA:64596 Definition: Catalysis of the reaction: a 1D-myo-inositol-1-phospho-N-[(R)-2-hydroxy-very-long-chain fatty acyl]-(R)-4-hydroxysphingoid base + GDP-alpha-D-mannose = an alpha-D-mannosyl-(1,6)-1D-myo-inositol-1-phospho-N-[(R)-2-hydroxy-very-long-chain fatty acyl]-(R)-4-hydroxysphingoid base + GDP + H+. Relationships: is a type of GO:0000030